carbon-halide lyase activity [GO:0016848] (molecular function) Relationships: is a type of GO:0016829 Definition: Catalysis of the breakage of a bond between carbon and any halogen atom. Subtypes: DDT-dehydrochlorinase activity [GO:0018833], dichloromethane dehalogenase activity [GO:0018834], 3-chloro-D-alanine dehydrochlorinase activity [GO:0019149], halohydrin hydrogen-halide-lyase activity [GO:0019181], GO:0047460, S-carboxymethylcysteine synthase activity [GO:0050272], L-propargylglycine synthase activity [GO:0062144], DIF dechlorinase activity [GO:0099085] Sources: GOC:mah